regulation of erythrocyte differentiation [GO:0045646] (biological process) Also known as: regulation of RBC differentiation, regulation of red blood cell differentiation Subtypes: regulation of definitive erythrocyte differentiation [GO:0010724], regulation of primitive erythrocyte differentiation [GO:0010725], negative regulation of erythrocyte differentiation [GO:0045647], positive regulation of erythrocyte differentiation [GO:0045648] Sources: GOC:go_curators Relationships: is a type of regulation of myeloid cell differentiation [GO:0045637]; regulates erythrocyte differentiation [GO:0030218] Definition: Any process that modulates the frequency, rate or extent of erythrocyte differentiation.